{
  "term_id": "GO:0046471",
  "gene": "UniProtKB:Q02509",
  "term_label": "phosphatidylglycerol metabolic process",
  "gene_symbol": "OC90",
  "gene_name": "Otoconin-90"
}